{
  "gene_name": "Small nuclear protein PRAC1",
  "gene": "UniProtKB:Q96KF2",
  "term_label": "Unknown molecular function",
  "term_id": "UNKNOWN:0001",
  "gene_symbol": "PRAC1"
}